{
  "gene_name": "Ataxin-2-like protein",
  "term_label": "cytoplasmic stress granule",
  "gene_symbol": "ATXN2L",
  "gene": "UniProtKB:Q8WWM7",
  "term_id": "GO:0010494"
}